mitochondrial ATP-gated potassium channel complex [GO:0062157] (CC) Definition: A protein-containing complex that is capable of the ATP-dependent diffusion of a potassium ion across the mitochondrial inner membrane. References: PMID:31435016 Relationships: is a type of potassium channel complex [GO:0034705]